{
  "term_id": "GO:0005634",
  "gene_name": "Ubiquitin-fold modifier 1",
  "gene": "UniProtKB:P61960",
  "term_label": "nucleus",
  "gene_symbol": "UFM1"
}